{
  "gene": "UniProtKB:Q96GK7",
  "gene_symbol": "FAHD2A",
  "term_label": "Unknown cellular component",
  "gene_name": "Fumarylacetoacetate hydrolase domain-containing protein 2A",
  "term_id": "UNKNOWN:0003"
}